{
  "term_label": "lipid droplet",
  "gene_name": "Lipid droplet-associated hydrolase",
  "gene_symbol": "LDAH",
  "term_id": "GO:0005811",
  "gene": "UniProtKB:Q9H6V9"
}